{
  "gene_symbol": "TIAM2",
  "gene": "UniProtKB:Q8IVF5",
  "gene_name": "Rho guanine nucleotide exchange factor TIAM2",
  "term_id": "GO:0005085",
  "term_label": "guanyl-nucleotide exchange factor activity"
}